{
  "gene_symbol": "CCDC149",
  "term_id": "UNKNOWN:0001",
  "gene": "UniProtKB:Q6ZUS6",
  "gene_name": "Coiled-coil domain-containing protein 149",
  "term_label": "Unknown molecular function"
}